stress response to zinc ion [GO:1990359] (biological process) References: PMID:17888400 Sources: GOC:kmv Definition: Any process that results in a change in state or activity of a cell or an organism (in terms of movement, secretion, enzyme production, gene expression, etc.) as a result of a disturbance in organismal or cellular homeostasis caused by a zinc ion stimulus. Relationships: is a type of response to zinc ion [GO:0010043]; is a type of stress response to metal ion [GO:0097501] Also known as: stress response to zinc, response to zinc ion stress, response to zinc toxicity